{
  "gene": "UniProtKB:Q9UFE4",
  "gene_symbol": "CCDC39",
  "term_id": "GO:0060285",
  "term_label": "cilium-dependent cell motility",
  "gene_name": "Coiled-coil domain-containing protein 39"
}